{
  "gene_symbol": "CFL2",
  "term_id": "GO:0015629",
  "term_label": "actin cytoskeleton",
  "gene_name": "Cofilin-2",
  "gene": "UniProtKB:Q9Y281"
}